establishment or maintenance of transmembrane electrochemical gradient [GO:0010248] (biological process) Relationships: is_a monoatomic ion transmembrane transport [GO:0034220] Sources: GOC:mah, GOC:sm Definition: The directed movement of ions to establish or maintain an electrochemical gradient across a membrane by means of some agent such as a transporter or pore.